{
  "term_id": "UNKNOWN:0002",
  "term_label": "Unknown biological process",
  "gene_symbol": "NSL1",
  "gene_name": "Kinetochore-associated protein NSL1 homolog",
  "gene": "UniProtKB:Q96IY1"
}